{
  "term_label": "chromatin organization",
  "gene": "UniProtKB:P06899",
  "term_id": "GO:0006325",
  "gene_name": "Histone H2B type 1-J",
  "gene_symbol": "H2BC11"
}